{
  "term_id": "UNKNOWN:0002",
  "gene_name": "ATP synthase subunit s, mitochondrial",
  "gene": "UniProtKB:Q99766",
  "term_label": "Unknown biological process",
  "gene_symbol": "DMAC2L"
}